xylan biosynthetic process [GO:0045492] (biological process) Subtypes: glucuronoxylan biosynthetic process [GO:0010417] Definition: The chemical reactions and pathways resulting in the formation of xylan, a polymer containing a beta-1,4-linked D-xylose backbone. Also known as: xylan anabolism, xylan biosynthesis, xylan formation, xylan synthesis References: PMID:11931668 Sources: GOC:go_curators Relationships: is a type of xylan metabolic process [GO:0045491]; is a type of cell wall polysaccharide biosynthetic process [GO:0070592]